{
  "gene_name": "Putative speedy protein E11",
  "term_id": "UNKNOWN:0003",
  "term_label": "Unknown cellular component",
  "gene": "UniProtKB:P0DTA3",
  "gene_symbol": "SPDYE11"
}